{
  "term_id": "UNKNOWN:0003",
  "gene": "UniProtKB:O14598",
  "gene_symbol": "VCY",
  "gene_name": "Testis-specific basic protein Y 1",
  "term_label": "Unknown cellular component"
}